atropine biosynthetic process [GO:1901051] (BP) Relationships: is a type of tropane alkaloid biosynthetic process [GO:0009710] Definition: The chemical reactions and pathways resulting in the formation of atropine. Atropine is the racemic mixture of hyoscyamine. References: PMID:2879005, PMID:33572199 Sources: GOC:TermGenie, GOC:yaf Also known as: atropine metabolic process, atropine metabolism, atropine anabolism, atropine biosynthesis, atropine formation, atropine synthesis, hyoscyamine biosynthetic process